{
  "gene": "UniProtKB:P02549",
  "term_label": "actin cytoskeleton organization",
  "gene_name": "Spectrin alpha chain, erythrocytic 1",
  "term_id": "GO:0030036",
  "gene_symbol": "SPTA1"
}